tryptophan 2-monooxygenase activity [GO:0050361] (molecular function) Sources: EC:1.13.12.3, RHEA:16165 Definition: Catalysis of the reaction: L-tryptophan + O2 = CO2 + H2O + indole-3-acetamide. Also known as: L-tryptophan:oxygen 2-oxidoreductase (decarboxylating) Relationships: is a type of GO:0016703